C-rich single-stranded DNA binding [GO:1990829] (MF) References: PMID:8127654 Relationships: is a type of GO:0003697 Definition: Binding to C-rich, single-stranded DNA. Also known as: C-rich ssDNA binding